{
  "gene": "UniProtKB:Q8WXI4",
  "gene_symbol": "ACOT11",
  "term_label": "long-chain fatty acyl-CoA hydrolase activity",
  "term_id": "GO:0052816",
  "gene_name": "Acyl-coenzyme A thioesterase 11"
}